{
  "term_label": "mannose metabolic process",
  "gene_name": "Phosphomannomutase 2",
  "term_id": "GO:0006013",
  "gene": "UniProtKB:O15305",
  "gene_symbol": "PMM2"
}